inositol hexakisphosphate kinase activity [GO:0000828] (molecular function) References: PMID:16429326 Sources: GOC:elh, GOC:vw Definition: Catalysis of the reaction: ATP + 1D-myo-inositol hexakisphosphate = ADP + diphospho-1D-myo-inositol-pentakisphosphate. The isomeric configuration of diphospho-1D-myo-inositol-pentakisphosphate (PP-IP5) is unknown. Also known as: IP6 kinase Subtypes: GO:0000830, inositol hexakisphosphate 6-kinase activity [GO:0000831], inositol hexakisphosphate 5-kinase activity [GO:0000832], inositol hexakisphosphate 1-kinase activity [GO:0052723], inositol hexakisphosphate 3-kinase activity [GO:0052724] Relationships: is a type of GO:0016776; is a type of inositol phosphate kinase activity [GO:0180030]